{
  "term_label": "guanyl-nucleotide exchange factor activity",
  "term_id": "GO:0005085",
  "gene_name": "RCC1-like G exchanging factor-like protein",
  "gene": "UniProtKB:Q96I51",
  "gene_symbol": "RCC1L"
}